{
  "gene_name": "Voltage-dependent calcium channel beta subunit-associated regulatory protein",
  "gene_symbol": "CBARP",
  "term_label": "plasma membrane",
  "term_id": "GO:0005886",
  "gene": "UniProtKB:Q8N350"
}